{
  "gene_name": "Omega-hydroxyceramide transacylase",
  "gene_symbol": "PNPLA1",
  "gene": "UniProtKB:Q8N8W4",
  "term_label": "cytoplasm",
  "term_id": "GO:0005737"
}